{
  "gene_symbol": "FBL",
  "term_id": "GO:0003723",
  "term_label": "RNA binding",
  "gene_name": "rRNA 2'-O-methyltransferase fibrillarin",
  "gene": "UniProtKB:P22087"
}